nonhomologous end joining complex [GO:0070419] (cellular component) Relationships: is a type of intracellular protein-containing complex [GO:0140535]; is a type of DNA repair complex [GO:1990391] Also known as: NHEJ complex, non-homologous end joining complex Subtypes: GO:0005958, DNA ligase IV complex [GO:0032807], GO:0070420 References: PMID:17072889, PMID:17938628 Sources: GOC:mah Definition: A protein complex that plays a role in DNA double-strand break repair via nonhomologous end joining. Such complexes typically contain a specialized DNA ligase (e.g. Lig4 in eukaryotes) and one or more proteins that bind to DNA ends.